{
  "gene_name": "Alanine--tRNA ligase, cytoplasmic",
  "term_label": "alanyl-tRNA aminoacylation",
  "term_id": "GO:0006419",
  "gene_symbol": "AARS1",
  "gene": "UniProtKB:P49588"
}